phosphatidylinositol-3,4-bisphosphate 3-phosphatase activity [GO:0051800] (molecular function) Also known as: PTEN activity Relationships: is a type of phosphatidylinositol-3,4-bisphosphate phosphatase activity [GO:0106017] Definition: Catalysis of the reaction: 1-phosphatidyl-1D-myo-inositol 3,4-bisphosphate + H2O = 1-phosphatidyl-1D-myo-inositol 4-phosphate + phosphate. References: PMID:9811831 Sources: GOC:bf